{
  "gene": "UniProtKB:Q5TC12",
  "gene_symbol": "ATPAF1",
  "gene_name": "ATP synthase mitochondrial F1 complex assembly factor 1",
  "term_label": "protein-containing complex stabilizing activity",
  "term_id": "GO:0140777"
}